{
  "term_id": "GO:0055085",
  "gene_name": "Solute carrier family 15 member 5",
  "gene_symbol": "SLC15A5",
  "gene": "UniProtKB:A6NIM6",
  "term_label": "transmembrane transport"
}